vomilenine reductase activity [GO:0050624] (molecular function) Definition: Catalysis of the reaction: 1,2-dihydrovomilenine + NADP+ = H+ + NADPH + vomilenine. Also known as: 1,2-dihydrovomilenine:NADP+ oxidoreductase activity Relationships: is a type of oxidoreductase activity, acting on the CH-NH group of donors, NAD or NADP as acceptor [GO:0016646] Sources: EC:1.5.1.32, RHEA:16409